{
  "gene_symbol": "ITGB1",
  "term_label": "laminin binding",
  "gene": "UniProtKB:P05556",
  "gene_name": "Integrin beta-1",
  "term_id": "GO:0043236"
}